chimeric non-reproductive fruiting body development [GO:0099136] (biological process) Subtypes: GO:0099134, altruistic, chimeric, non-reproductive fruiting body development [GO:0099137] Relationships: is a type of GO:0099135 References: PMID:18272966 Definition: Development of a non-reproductive fruiting body formed by aggregation of cells with different genotypes.